{
  "gene_name": "G-protein coupled receptor 157",
  "term_id": "GO:0004930",
  "gene_symbol": "GPR157",
  "term_label": "G protein-coupled receptor activity",
  "gene": "UniProtKB:Q5UAW9"
}